{
  "term_id": "GO:0051963",
  "gene_symbol": "OPCML",
  "gene": "UniProtKB:Q14982",
  "term_label": "regulation of synapse assembly",
  "gene_name": "Opioid-binding protein_cell adhesion molecule"
}